oligosaccharide metabolic process [GO:0009311] (biological process) Relationships: is a type of carbohydrate metabolic process [GO:0005975] Definition: The chemical reactions and pathways involving oligosaccharides, molecules with between two and (about) 20 monosaccharide residues connected by glycosidic linkages. Also known as: oligosaccharide metabolism, multicellular organismal oligosaccharide metabolic process Subtypes: disaccharide metabolic process [GO:0005984], oligosaccharide biosynthetic process [GO:0009312], oligosaccharide catabolic process [GO:0009313], raffinose metabolic process [GO:0033530], GO:0033531, cellodextrin metabolic process [GO:2000889], cellotriose metabolic process [GO:2000893], GO:2000900, GO:2000902, maltoheptaose metabolic process [GO:2001122] Sources: ISBN:0198506732